{
  "gene_symbol": "CXCL14",
  "gene_name": "C-X-C motif chemokine 14",
  "term_id": "UNKNOWN:0003",
  "gene": "UniProtKB:O95715",
  "term_label": "Unknown cellular component"
}